{
  "gene_symbol": "CATIP",
  "gene": "UniProtKB:Q7Z7H3",
  "gene_name": "Ciliogenesis-associated TTC17-interacting protein",
  "term_id": "GO:0030041",
  "term_label": "actin filament polymerization"
}